{
  "gene": "UniProtKB:Q9Y337",
  "gene_name": "Kallikrein-5",
  "term_label": "secretory granule",
  "term_id": "GO:0030141",
  "gene_symbol": "KLK5"
}